{
  "gene": "UniProtKB:Q9UIG0",
  "term_id": "GO:0042393",
  "gene_name": "Tyrosine-protein kinase BAZ1B",
  "gene_symbol": "BAZ1B",
  "term_label": "histone binding"
}